{
  "gene_name": "Oxidized purine nucleoside triphosphate hydrolase",
  "term_label": "cytoplasm",
  "term_id": "GO:0005737",
  "gene_symbol": "NUDT1",
  "gene": "UniProtKB:P36639"
}